positive regulation of mating projection assembly [GO:1902917] (biological process) Definition: Any process that activates or increases the frequency, rate or extent of mating projection assembly. References: PMID:12455985 Sources: GOC:TermGenie, GOC:di, GO_REF:0000058 Relationships: is a type of GO:0031383; is a type of positive regulation of developmental process [GO:0051094]; is a type of positive regulation of plasma membrane bounded cell projection assembly [GO:0120034]; is part of positive regulation of conjugation with cellular fusion [GO:0031139]; positively regulates mating projection formation [GO:0031382] Also known as: up regulation of mating projection assembly, up-regulation of mating projection assembly, upregulation of mating projection assembly, activation of mating projection assembly, activation of mating projection biogenesis, positive regulation of mating projection biogenesis, up regulation of mating projection biogenesis, up-regulation of mating projection biogenesis, upregulation of mating projection biogenesis